{
  "gene_name": "WAS protein family homolog 6",
  "term_label": "retrograde transport, endosome to Golgi",
  "gene": "UniProtKB:Q9NQA3",
  "gene_symbol": "WASH6P",
  "term_id": "GO:0042147"
}